{
  "term_id": "GO:0000278",
  "term_label": "mitotic cell cycle",
  "gene": "UniProtKB:P68363",
  "gene_symbol": "TUBA1B",
  "gene_name": "Tubulin alpha-1B chain"
}